protein phosphatase 1 binding [GO:0008157] (molecular function) Relationships: is a type of protein phosphatase binding [GO:0019903] Definition: Binding to a protein phosphatase 1. Sources: GOC:jl